{
  "term_label": "MHC class I peptide loading complex",
  "gene_name": "Tapasin",
  "gene_symbol": "TAPBP",
  "gene": "UniProtKB:O15533",
  "term_id": "GO:0042824"
}